{
  "term_id": "GO:0005634",
  "gene_symbol": "SKI",
  "term_label": "nucleus",
  "gene_name": "Ski oncogene",
  "gene": "UniProtKB:P12755"
}